caffeine synthase activity [GO:0102741] (MF) Sources: EC:2.1.1.160 Definition: Catalysis of the reaction: 1,7-dimethylxanthine + S-adenosyl-L-methionine = H+ + caffeine + S-adenosyl-L-homocysteine. Also converts theobromine to caffeine and 7-methylxanthine to theobromine. Relationships: is a type of methyltransferase activity [GO:0008168] Also known as: paraxanthine:S-adenosyl-L-methionine 3-N-methyltransferase activity, theobromine:S-adenosyl-L-methionine 1-N-methyltransferase activity, 3N-methyltransferase activity, dimethylxanthine methyltransferase activity